CAMKK-AMPK signaling cascade [GO:0061762] (biological process) Regulation: regulated by regulation of CAMKK-AMPK signaling cascade [GO:1905289]; negatively regulated by GO:1905290; positively regulated by positive regulation of CAMKK-AMPK signaling cascade [GO:1905291] Also known as: stress-activated AMP-activated protein kinase signaling cascade Relationships: is a type of GO:0019722; has part AMP-activated protein kinase activity [GO:0004679]; has part calcium/calmodulin-dependent protein kinase activity [GO:0004683]; BFO_0000051 calcium ion binding [GO:0005509]; has part GO:0005516 Definition: The series of molecular signals in which calmodulin-dependent protein kinase activity enabled by a CAMKK directly activates an AMPK. The cascade begins with calmodulin binding calcium which in turn binds CAMKK enabling its calmodulin-dependent protein kinase activity. The cascade ends with AMP-activated protein kinase activity. References: PMID:23010169, PMID:24709372 Sources: GOC:PARL, GOC:dph, GOC:pad